{
  "gene_symbol": "RASGRP3",
  "gene": "UniProtKB:Q8IV61",
  "term_id": "GO:0007265",
  "gene_name": "Ras guanyl-releasing protein 3",
  "term_label": "Ras protein signal transduction"
}